{
  "gene_name": "Histone-lysine N-methyltransferase SETD2",
  "gene": "UniProtKB:Q9BYW2",
  "term_id": "GO:0046975",
  "term_label": "histone H3K36 methyltransferase activity",
  "gene_symbol": "SETD2"
}